glutathione-dependent sulfide quinone oxidoreductase activity [GO:0106436] (molecular function) Definition: Catalysis of the reaction: a quinone + glutathione + H+ + hydrogen sulfide = a quinol + S-sulfanylglutathione. Sources: RHEA:55156 Also known as: eukaryotic sulfide quinone oxidoreductase Relationships: is_a oxidoreductase activity, acting on a sulfur group of donors, quinone or similar compound as acceptor [GO:0016672]